{
  "gene": "UniProtKB:O43490",
  "term_label": "camera-type eye photoreceptor cell differentiation",
  "term_id": "GO:0060219",
  "gene_name": "Prominin-1",
  "gene_symbol": "PROM1"
}